acyl-CoA (9+3)-desaturase activity [GO:0102985] (molecular function) Also known as: delta12-fatty-acid desaturase activity Sources: EC:1.14.19.6 Definition: Catalysis of the introduction of a cis double bond at position 12 of fatty-acyl-CoAs that contain a cis double bond at position 9. Specific reactions include: (9Z)-hexadecenoyl-CoA + 2 Fe(II)-[cytochrome b5] + 2 H+ + O2 = (9Z,12Z)-hexadecadienoyl-CoA + 2 Fe(III)-[cytochrome b5] + 2 H2O; and (9Z)-hexadecenoyl-CoA + 2 Fe(II)-[cytochrome b5] + O2 + 2 H(+) = (9Z,12Z)-hexadecadienoyl-CoA + 2 Fe(III)-[cytochrome b5] + 2 H2O. Relationships: is a type of acyl-CoA desaturase activity [GO:0016215]